{
  "term_id": "GO:0006898",
  "gene_name": "C-type mannose receptor 2",
  "gene_symbol": "MRC2",
  "gene": "UniProtKB:Q9UBG0",
  "term_label": "receptor-mediated endocytosis"
}